{
  "term_id": "GO:0090443",
  "term_label": "FAR/SIN/STRIPAK complex",
  "gene_symbol": "PDCD10",
  "gene_name": "Programmed cell death protein 10",
  "gene": "UniProtKB:Q9BUL8"
}